oxidative phosphorylation uncoupler activity [GO:0017077] (molecular function) References: PMID:15738989, PMID:16179945 Regulation: positively regulated by positive regulation of oxidative phosphorylation uncoupler activity [GO:2000277] Definition: Enables the transfer of protons from mitochondrial intermembrane space into mitochondrial matrix, dissipating the proton gradient across the mitochondrial inner membrane established by the electron transport chain during the oxidative phosphorylation (proton leak). Proton leak uncouples the processes of electron transport/proton generation and ATP synthesis. Also known as: mitochondrial uncoupling protein activity, uncoupling protein activity Relationships: is a type of transmembrane transporter activity [GO:0022857]; is part of GO:1902600